{
  "term_id": "GO:0006694",
  "gene_symbol": "STAR",
  "gene_name": "Steroidogenic acute regulatory protein, mitochondrial",
  "gene": "UniProtKB:P49675",
  "term_label": "steroid biosynthetic process"
}